negative regulation of complement activation [GO:0045916] (biological process) Definition: Any process that stops, prevents, or reduces the frequency, rate or extent of complement activation. Relationships: is_a negative regulation of immune effector process [GO:0002698]; is a type of GO:0002921; is a type of regulation of complement activation [GO:0030449]; negatively regulates complement activation [GO:0006956] Also known as: down regulation of complement activation, down-regulation of complement activation, downregulation of complement activation, negative regulation of complement cascade, inhibition of complement activation Subtypes: negative regulation of complement activation, lectin pathway [GO:0001869], negative regulation of activation of membrane attack complex [GO:0001971], negative regulation of complement activation, alternative pathway [GO:0045957], GO:0045959 Sources: GOC:go_curators